(Z)-nonadeca-1,14-diene biosynthetic process [GO:1900879] (biological process) Definition: The chemical reactions and pathways resulting in the formation of (Z)-nonadeca-1,14-diene. Sources: GOC:TermGenie, GOC:mengo_curators Also known as: (Z)-nonadeca-1,14-diene anabolism, (Z)-nonadeca-1,14-diene biosynthesis, (Z)-nonadeca-1,14-diene formation, (Z)-nonadeca-1,14-diene synthesis Relationships: is a type of olefin biosynthetic process [GO:1900674]; is a type of (Z)-nonadeca-1,14-diene metabolic process [GO:1900878] Regulation: regulated by GO:1900941; negatively regulated by negative regulation of (Z)-nonadeca-1,14-diene biosynthetic process [GO:1900942]; positively regulated by positive regulation of (Z)-nonadeca-1,14-diene biosynthetic process [GO:1900943]